{
  "term_id": "GO:0070325",
  "term_label": "lipoprotein particle receptor binding",
  "gene_symbol": "RELN",
  "gene_name": "Reelin",
  "gene": "UniProtKB:P78509"
}